subpellicular network [GO:0020038] (CC) References: PMID:11420112 Relationships: is a type of cellular anatomical structure [GO:0110165]; is part of GO:0005856; is part of GO:0020039 Definition: A mechanically stable cytoskeletal structure associated with the cytoplasmic face of the pellicle and surrounding the microtubule-based cytoskeleton.